interleukin-28B production [GO:0072629] (biological process) Also known as: IL-28B production, IL28B production, interferon lambda 3 production, interleukin-28B secretion Note: Note that this term is in the subset of terms that should not be used for direct gene product annotation. Instead, select one of the 'regulation' children terms. References: PMID:15546383 Sources: GOC:BHF, GOC:mah Relationships: is a type of type III interferon production [GO:0034343] Definition: The appearance of interleukin-28B due to biosynthesis or secretion following a cellular stimulus, resulting in an increase in its intracellular or extracellular levels.